{
  "term_id": "GO:0005923",
  "term_label": "bicellular tight junction",
  "gene": "UniProtKB:O95471",
  "gene_name": "Claudin-7",
  "gene_symbol": "CLDN7"
}